{
  "gene_name": "Ubiquitin-associated and SH3 domain-containing protein B",
  "gene_symbol": "UBASH3B",
  "term_label": "regulation of osteoclast differentiation",
  "term_id": "GO:0045670",
  "gene": "UniProtKB:Q8TF42"
}